adenosylcobinamide hydrolase activity [GO:0043756] (molecular function) Sources: EC:3.5.1.90, RHEA:23504 Also known as: AdoCbi amidohydrolase activity, AdoCbi hydrolase activity, CbiZ, adenosylcobinamide amidohydrolase activity Relationships: is a type of GO:0016811 Definition: Catalysis of the reaction: adenosylcobinamide + H2O = (R)-1-aminopropan-2-ol + adenosylcobyrate.